{
  "term_label": "plasma membrane",
  "term_id": "GO:0005886",
  "gene_symbol": "GRIK2",
  "gene": "UniProtKB:Q13002",
  "gene_name": "Glutamate receptor ionotropic, kainate 2"
}